{
  "gene_symbol": "RSPH3",
  "term_id": "UNKNOWN:0001",
  "term_label": "Unknown molecular function",
  "gene": "UniProtKB:Q86UC2",
  "gene_name": "Radial spoke head protein 3 homolog"
}